{
  "term_label": "complement component C5a receptor activity",
  "gene": "UniProtKB:P21730",
  "gene_symbol": "C5AR1",
  "gene_name": "C5a anaphylatoxin chemotactic receptor 1",
  "term_id": "GO:0004878"
}